{
  "term_id": "UNKNOWN:0003",
  "term_label": "Unknown cellular component",
  "gene_name": "Spermatogenesis-associated protein 31A7",
  "gene_symbol": "SPATA31A7",
  "gene": "UniProtKB:Q8IWB4"
}